{
  "term_id": "GO:0006954",
  "gene_name": "C-C chemokine receptor type 3",
  "gene_symbol": "CCR3",
  "gene": "UniProtKB:P51677",
  "term_label": "inflammatory response"
}